{
  "gene": "UniProtKB:Q6MZM0",
  "gene_name": "Ferroxidase HEPHL1",
  "term_label": "Unknown biological process",
  "gene_symbol": "HEPHL1",
  "term_id": "UNKNOWN:0002"
}